{
  "gene": "UniProtKB:P51808",
  "term_id": "GO:0005868",
  "gene_symbol": "DYNLT3",
  "term_label": "cytoplasmic dynein complex",
  "gene_name": "Dynein light chain Tctex-type 3"
}